{
  "gene_name": "Cyclin-dependent kinase 14",
  "gene_symbol": "CDK14",
  "term_id": "GO:0030332",
  "gene": "UniProtKB:O94921",
  "term_label": "cyclin binding"
}